{
  "gene": "UniProtKB:Q16270",
  "term_id": "GO:0001525",
  "gene_symbol": "IGFBP7",
  "term_label": "angiogenesis",
  "gene_name": "Insulin-like growth factor-binding protein 7"
}